epicardium morphogenesis [GO:1905223] (biological process) Relationships: is a type of anatomical structure morphogenesis [GO:0009653] References: PMID:18718461 Sources: GOC:BHF, GOC:TermGenie, GOC:rl, GO_REF:0000083 Also known as: heart epicardium morphogenesis, visceral serous pericardium of heart morphogenesis, visceral serous pericardium proper morphogenesis, pericardium visceral mesothelium morphogenesis Definition: The developmental process by which an epicardium is generated and organized.